{
  "gene_symbol": "CD2",
  "gene": "UniProtKB:P06729",
  "term_id": "GO:0030101",
  "term_label": "natural killer cell activation",
  "gene_name": "T-cell surface antigen CD2"
}